{
  "gene": "UniProtKB:Q9UK11",
  "gene_symbol": "ZNF223",
  "term_id": "UNKNOWN:0002",
  "term_label": "Unknown biological process",
  "gene_name": "Zinc finger protein 223"
}